{
  "term_id": "GO:0005615",
  "gene": "UniProtKB:Q9BZD7",
  "gene_symbol": "PRRG3",
  "term_label": "extracellular space",
  "gene_name": "Transmembrane gamma-carboxyglutamic acid protein 3"
}